negative regulation of endopeptidase activity [GO:0010951] (biological process) Definition: Any process that decreases the frequency, rate or extent of endopeptidase activity, the endohydrolysis of peptide bonds within proteins. Sources: GOC:dph, GOC:tb Subtypes: negative regulation of serine-type endopeptidase activity [GO:1900004] Relationships: is_a negative regulation of peptidase activity [GO:0010466]; is a type of regulation of endopeptidase activity [GO:0052548]; negatively regulates endopeptidase activity [GO:0004175]